{
  "gene_symbol": "SRXN1",
  "term_id": "GO:0032542",
  "term_label": "sulfiredoxin activity",
  "gene": "UniProtKB:Q9BYN0",
  "gene_name": "Sulfiredoxin-1"
}